{
  "gene_name": "N-acetyllactosaminide beta-1,6-N-acetylglucosaminyl-transferase",
  "gene_symbol": "GCNT2",
  "gene": "UniProtKB:Q8N0V5",
  "term_label": "Unknown cellular component",
  "term_id": "UNKNOWN:0003"
}